chorismate mutase activity [GO:0004106] (molecular function) Sources: EC:5.4.99.5, RHEA:13897 Also known as: hydroxyphenylpyruvate synthase activity, chorismate pyruvatemutase activity Definition: Catalysis of the reaction: chorismate = prephenate. Relationships: is a type of GO:0016866